{
  "gene_symbol": "GPC5",
  "term_label": "cell migration",
  "gene": "UniProtKB:P78333",
  "term_id": "GO:0016477",
  "gene_name": "Glypican-5"
}